GAIT complex [GO:0097452] (cellular component) Also known as: IFN-gamma-activated inhibitor of translation complex, gamma interferon-activated inhibitor of translation complex Relationships: is a type of protein-containing complex [GO:0032991] References: PMID:15479637, PMID:23071094 Sources: GOC:br Definition: A protein complex which mediates interferon-gamma-induced transcript-selective translation inhibition in inflammation processes. The complex binds to stem loop-containing GAIT elements in the 3'-UTR of diverse inflammatory mRNAs and suppresses their translation by blocking the recruitment of the 43S ribosomal complex to m7G cap-bound eIF4G. In humans it includes RPL13A, EPRS, SYNCRIP and GAPDH; mouse complexes lack SYNCRIP.